ABC-type oligopeptide transporter activity [GO:0015421] (molecular function) Also known as: ABC-type oligopeptide transporter, ATP-dependent oligopeptide transmembrane transporter activity, oligopeptide ABC transporter, ATPase-coupled oligopeptide transmembrane transporter activity, oligopeptide permease activity, oligopeptide-transporting ATPase activity Sources: RHEA:14429 Definition: Catalysis of the reaction: ATP + H2O + oligopeptide(out) = ADP + phosphate + oligopeptide(in). Relationships: is a type of oligopeptide transmembrane transporter activity [GO:0035673]; is a type of ABC-type transporter activity [GO:0140359]